regulation of B cell proliferation [GO:0030888] (biological process) Relationships: is a type of regulation of lymphocyte proliferation [GO:0050670]; is a type of regulation of B cell activation [GO:0050864]; regulates B cell proliferation [GO:0042100] Also known as: regulation of B lymphocyte proliferation, regulation of B-cell proliferation, regulation of B-lymphocyte proliferation Sources: GOC:mah Subtypes: GO:0030889, positive regulation of B cell proliferation [GO:0030890] Definition: Any process that modulates the frequency, rate or extent of B cell proliferation.